{
  "gene": "UniProtKB:O00220",
  "gene_name": "Tumor necrosis factor receptor superfamily member 10A",
  "term_id": "GO:0036462",
  "term_label": "TRAIL-activated apoptotic signaling pathway",
  "gene_symbol": "TNFRSF10A"
}